{
  "term_label": "Unknown molecular function",
  "gene_name": "Protein FAM90A17",
  "gene_symbol": "FAM90A17",
  "gene": "UniProtKB:P0DV74",
  "term_id": "UNKNOWN:0001"
}